{
  "gene_name": "Somatostatin receptor type 1",
  "term_label": "neuropeptide binding",
  "gene_symbol": "SSTR1",
  "term_id": "GO:0042923",
  "gene": "UniProtKB:P30872"
}